{
  "term_label": "plasma membrane",
  "gene_name": "Protocadherin Fat 4",
  "gene": "UniProtKB:Q6V0I7",
  "gene_symbol": "FAT4",
  "term_id": "GO:0005886"
}